{
  "term_id": "GO:0005634",
  "gene_name": "DNA-binding protein RFX6",
  "term_label": "nucleus",
  "gene_symbol": "RFX6",
  "gene": "UniProtKB:Q8HWS3"
}